formation of radial glial scaffolds [GO:0021943] (biological process) References: PMID:15157725 Sources: GOC:cls, GOC:dgh, GOC:dph, GOC:jid, GO_REF:0000021 Definition: The formation of scaffolds from a radial glial cell. The scaffolds are used as a substrate for the radial migration of cells. Relationships: is_a cell morphogenesis [GO:0000902]; is part of hindbrain radial glia guided cell migration [GO:0021932] Regulation: RO_0002211 by regulation of formation of radial glial scaffolds [GO:0061924]; RO_0002212 by negative regulation of formation of radial glial scaffolds [GO:0061925]; positively regulated by positive regulation of formation of radial glial scaffolds [GO:0061926] Also known as: Bergmann fiber biosynthesis, Bergmann fiber formation